{
  "gene": "UniProtKB:O75871",
  "term_id": "GO:0007165",
  "gene_name": "Carcinoembryonic antigen-related cell adhesion molecule 4",
  "gene_symbol": "CEACAM4",
  "term_label": "signal transduction"
}